{
  "term_label": "calcium ion binding",
  "term_id": "GO:0005509",
  "gene_name": "Neurocalcin-delta",
  "gene_symbol": "NCALD",
  "gene": "UniProtKB:P61601"
}